symbiont-mediated suppression of host type I interferon-mediated signaling pathway [GO:0039502] (biological process) Definition: A process in which a symbiont interferes with, inhibits or disrupts a type I interferon-mediated signaling in the host organism. Type I interferons include the interferon-alpha, beta, delta, episilon, zeta, kappa, tau, and omega gene families. Relationships: is a type of GO:0140886 References: PMID:19802576, PMID:26712804, PMID:32464097, PMID:32733001, PMID:33097660 Sources: GOC:add, GOC:bf, GOC:sp Also known as: negative regulation by virus of host type I interferon-mediated signaling pathway, suppression by virus of host type I IFN-mediated signaling pathway, suppression by virus of host type I interferon-mediated signalling pathway, suppression by virus of host type I interferon-mediated signaling pathway, inhibition of host interferon signaling pathway by virus